ligand-gated monoatomic ion channel activity involved in regulation of presynaptic membrane potential [GO:0099507] (molecular function) References: PMID:15145529, PMID:19558451 Sources: GOC:dos Definition: Any ligand-gated ion channel activity, occurring in the presynaptic membrane, that is involved in regulation of presynaptic membrane potential. Also known as: ligand-gated ion channel activity involved in regulation of presynaptic membrane potential, ligand gated ion channel activity involved in regulation of presynaptic membrane potential, ligand-dependent ion channel activity involved in regulation of pre-synaptic membrane potential, ligand-dependent ion channel activity involved in regulation of presynaptic membrane potential, ligand-gated ion channel activity involved in regulation of pre-synaptic membrane potential Relationships: is a type of ligand-gated monoatomic ion channel activity [GO:0015276]; BFO_0000050 regulation of presynaptic membrane potential [GO:0099505]; occurs in presynaptic membrane [GO:0042734]